{
  "gene_name": "B-cell linker protein",
  "term_label": "cell surface receptor protein tyrosine kinase signaling pathway",
  "gene_symbol": "BLNK",
  "gene": "UniProtKB:Q8WV28",
  "term_id": "GO:0007169"
}